{
  "gene_symbol": "JAK3",
  "term_label": "growth hormone receptor signaling pathway via JAK-STAT",
  "gene_name": "Tyrosine-protein kinase JAK3",
  "gene": "UniProtKB:P52333",
  "term_id": "GO:0060397"
}